root epithelial mucilage biosynthetic process [GO:0048356] (biological process) Also known as: root epithelial mucilage anabolism, root epithelial mucilage biosynthesis, root epithelial mucilage formation, root epithelial mucilage synthesis Definition: The chemical reactions and pathways resulting in the formation of mucilage that occur in the root epithelium; mucilage is normally synthesized during root growth. Sources: GOC:jid Relationships: is a type of mucilage biosynthetic process [GO:0010192]